{
  "term_label": "nucleus",
  "gene_symbol": "MDFIC",
  "term_id": "GO:0005634",
  "gene_name": "MyoD family inhibitor domain-containing protein",
  "gene": "UniProtKB:Q9P1T7"
}